{
  "gene": "UniProtKB:Q15120",
  "term_label": "regulation of glucose metabolic process",
  "gene_name": "[Pyruvate dehydrogenase (acetyl-transferring)] kinase isozyme 3, mitochondrial",
  "gene_symbol": "PDK3",
  "term_id": "GO:0010906"
}